{
  "gene": "UniProtKB:Q8NCU8",
  "term_id": "UNKNOWN:0001",
  "gene_name": "Mitoregulin",
  "gene_symbol": "MTLN",
  "term_label": "Unknown molecular function"
}